positive regulation of protein desumoylation [GO:0060189] (biological process) Sources: GOC:dph, GOC:tb Definition: Any process that increases the frequency, rate or extent of protein desumoylation. Protein desumoylation is the process in which a SUMO protein (small ubiquitin-related modifier) is cleaved from its target protein. Relationships: is a type of regulation of protein desumoylation [GO:0060188]; is a type of GO:1903322; positively regulates protein desumoylation [GO:0016926]